{
  "gene_symbol": "SCRN2",
  "gene": "UniProtKB:Q96FV2",
  "term_label": "Unknown cellular component",
  "gene_name": "Secernin-2",
  "term_id": "UNKNOWN:0003"
}